{
  "gene": "UniProtKB:Q7Z2E3",
  "term_label": "mismatched DNA binding",
  "term_id": "GO:0030983",
  "gene_name": "Aprataxin",
  "gene_symbol": "APTX"
}